{
  "gene": "UniProtKB:Q9P218",
  "gene_symbol": "COL20A1",
  "gene_name": "Collagen alpha-1(XX) chain",
  "term_id": "UNKNOWN:0002",
  "term_label": "Unknown biological process"
}